{
  "gene": "UniProtKB:Q9BWF3",
  "gene_name": "RNA-binding protein 4",
  "term_label": "regulation of alternative mRNA splicing, via spliceosome",
  "gene_symbol": "RBM4",
  "term_id": "GO:0000381"
}